{
  "term_label": "ephrin receptor signaling pathway",
  "term_id": "GO:0048013",
  "gene": "UniProtKB:P52799",
  "gene_name": "Ephrin-B2",
  "gene_symbol": "EFNB2"
}